{
  "gene_name": "Ubiquitin conjugation factor E4 B",
  "gene_symbol": "UBE4B",
  "term_id": "GO:0005737",
  "gene": "UniProtKB:O95155",
  "term_label": "cytoplasm"
}